{
  "term_id": "GO:0005777",
  "gene_symbol": "CRAT",
  "gene": "UniProtKB:P43155",
  "term_label": "peroxisome",
  "gene_name": "Carnitine O-acetyltransferase"
}